{
  "gene_symbol": "ZNF318",
  "gene_name": "Zinc finger protein 318",
  "term_id": "GO:0045892",
  "gene": "UniProtKB:Q5VUA4",
  "term_label": "negative regulation of DNA-templated transcription"
}